{
  "gene_name": "Cysteine-rich secretory protein 1",
  "term_id": "UNKNOWN:0001",
  "gene": "UniProtKB:P54107",
  "term_label": "Unknown molecular function",
  "gene_symbol": "CRISP1"
}